{
  "term_id": "UNKNOWN:0002",
  "gene": "UniProtKB:A6NKP2",
  "gene_name": "Putative short-chain dehydrogenase_reductase family 42E member 2",
  "term_label": "Unknown biological process",
  "gene_symbol": "SDR42E2"
}